lipoxygenase pathway [GO:0019372] (biological process) Relationships: is a type of fatty acid metabolic process [GO:0006631]; is a type of icosanoid metabolic process [GO:0006690] Subtypes: green leaf volatile biosynthetic process [GO:0010597] References: PMID:17163881 Sources: GOC:mah Definition: The chemical reactions and pathways by which an unsaturated fatty acid (such as arachidonic acid or linolenic acid) is converted to other compounds, and in which the first step is hydroperoxide formation catalyzed by lipoxygenase.